{
  "gene_symbol": "CRACR2B",
  "term_label": "Unknown cellular component",
  "gene": "UniProtKB:Q8N4Y2",
  "term_id": "UNKNOWN:0003",
  "gene_name": "EF-hand calcium-binding domain-containing protein 4A"
}